{
  "gene_symbol": "AUP1",
  "term_id": "GO:0005789",
  "gene": "UniProtKB:Q9Y679",
  "gene_name": "Lipid droplet-regulating VLDL assembly factor AUP1",
  "term_label": "endoplasmic reticulum membrane"
}